histone H3T45 kinase activity [GO:0140857] (molecular function) Definition: Catalysis of the reaction: histone H3-threonine (position 45) + ATP = histone H3-phosphothreonine (position 45) + ADP. This reaction is the addition of a phosphate group to the threonine residue at position 45 of histone H3. Also known as: histone kinase activity (H3-T45 specific), histone threonine kinase activity (H3-T45 specific), histone-threonine kinase activity (H3-T45 specific) References: PMID:24820035 Relationships: is a type of protein serine/threonine kinase activity [GO:0004674]; is a type of histone H3 kinase activity [GO:0140996] Note: Comment: Note that the residue position corresponds to the canonical human H3 histone (UniProtKB:P84243); this residue is conserved across all eukaryotes. Residue 1 is the first residue following removal of the initiating Methionine (Met). Note that each histone is encoded by multiple genes, and sequences may vary across different genes within an organism.